GAU codon-amino acid adaptor activity [GO:0033457] (molecular function) Note: Note that in the standard genetic code, GAT codes for aspartic acid. Sources: GOC:mah Relationships: is a type of GO:0030533 Also known as: GAT codon-amino acid adaptor activity, aspartic acid tRNA Definition: A triplet codon-amino acid adaptor activity that recognizes a GAU codon.